negative regulation of [4Fe-4S] cluster assembly [GO:1900492] (biological process) Relationships: is a type of GO:1900491; is a type of negative regulation of iron-sulfur cluster assembly [GO:1903330]; negatively regulates GO:0044572 Also known as: down regulation of 4Fe-4S cluster assembly, down regulation of [4Fe-4S] cluster assembly, down-regulation of 4Fe-4S cluster assembly, down-regulation of [4Fe-4S] cluster assembly, downregulation of 4Fe-4S cluster assembly, downregulation of [4Fe-4S] cluster assembly, negative regulation of 4Fe-4S cluster assembly, inhibition of 4Fe-4S cluster assembly, inhibition of [4Fe-4S] cluster assembly, down regulation of [4Fe-4S] cluster biosynthetic process, down-regulation of [4Fe-4S] cluster biosynthetic process, downregulation of [4Fe-4S] cluster biosynthetic process, inhibition of [4Fe-4S] cluster biosynthetic process, negative regulation of [4Fe-4S] cluster biosynthetic process Definition: Any process that stops, prevents or reduces the frequency, rate or extent of [4Fe-4S] cluster assembly. Sources: GOC:TermGenie, GOC:mengo_curators, GOC:pr